{
  "gene": "UniProtKB:O75146",
  "term_id": "GO:0048268",
  "term_label": "clathrin coat assembly",
  "gene_symbol": "HIP1R",
  "gene_name": "Huntingtin-interacting protein 1-related protein"
}